{
  "gene": "UniProtKB:O75333",
  "term_id": "GO:0001708",
  "gene_symbol": "TBX10",
  "term_label": "cell fate specification",
  "gene_name": "T-box transcription factor TBX10"
}